cyanuric acid catabolic process [GO:0042200] (biological process) Definition: The chemical reactions and pathways resulting in the breakdown of cyanuric acid, a potential degradation product of triazine herbicides. Sources: UM-BBD_pathwayID:cya Relationships: is a type of s-triazine compound catabolic process [GO:0042204] Also known as: cyanuric acid breakdown, cyanuric acid catabolism, cyanuric acid degradation